{
  "gene_symbol": "TBC1D22A",
  "term_id": "UNKNOWN:0002",
  "term_label": "Unknown biological process",
  "gene": "UniProtKB:Q8WUA7",
  "gene_name": "TBC1 domain family member 22A"
}